{
  "term_label": "cell-cell adhesion",
  "gene_name": "LIM and senescent cell antigen-like-containing domain protein 1",
  "gene": "UniProtKB:P48059",
  "term_id": "GO:0098609",
  "gene_symbol": "LIMS1"
}